{
  "gene_symbol": "ALOX15B",
  "term_label": "Unknown cellular component",
  "gene_name": "Polyunsaturated fatty acid lipoxygenase ALOX15B",
  "term_id": "UNKNOWN:0003",
  "gene": "UniProtKB:O15296"
}